enamel mineralization [GO:0070166] (biological process) Definition: The process in which calcium salts, mainly carbonated hydroxyapatite, are deposited in tooth enamel. Also known as: enamel formation References: PMID:10206335, PMID:16931858, PMID:21196346 Sources: GOC:BHF, GOC:mah, GOC:sl Relationships: is a type of tooth mineralization [GO:0034505]; is part of GO:0097186 Regulation: regulated by regulation of enamel mineralization [GO:0070173]; negatively regulated by negative regulation of enamel mineralization [GO:0070174]; positively regulated by GO:0070175